{
  "gene_symbol": "HNRNPAB",
  "gene": "UniProtKB:Q99729",
  "term_id": "GO:0010468",
  "term_label": "regulation of gene expression",
  "gene_name": "Heterogeneous nuclear ribonucleoprotein A_B"
}